{
  "gene_name": "Golgin subfamily A member 8Q",
  "term_label": "cis-Golgi network",
  "term_id": "GO:0005801",
  "gene_symbol": "GOLGA8Q",
  "gene": "UniProtKB:H3BV12"
}